regulation of autophagy [GO:0010506] (biological process) Definition: Any process that modulates the frequency, rate or extent of autophagy. Autophagy is the process in which cells digest parts of their own cytoplasm. Sources: GOC:dph, GOC:tb Subtypes: GO:0010507, GO:0010508, regulation of macroautophagy [GO:0016241], GO:0140505, regulation of autophagy of mitochondrion [GO:1903146], regulation of chaperone-mediated autophagy [GO:1904714] Relationships: is a type of regulation of catabolic process [GO:0009894]; regulates GO:0006914